{
  "gene_symbol": "CHRNA3",
  "gene_name": "Neuronal acetylcholine receptor subunit alpha-3",
  "term_label": "monoatomic ion transmembrane transport",
  "gene": "UniProtKB:P32297",
  "term_id": "GO:0034220"
}